{
  "term_label": "protein auto-ADP-ribosylation",
  "gene": "UniProtKB:Q7Z3E1",
  "gene_symbol": "TIPARP",
  "term_id": "GO:0070213",
  "gene_name": "Protein mono-ADP-ribosyltransferase TIPARP"
}